{
  "term_label": "GTP binding",
  "gene_symbol": "ARL3",
  "gene": "UniProtKB:P36405",
  "term_id": "GO:0005525",
  "gene_name": "ADP-ribosylation factor-like protein 3"
}